{
  "term_id": "GO:0017075",
  "gene": "UniProtKB:Q8NB66",
  "gene_symbol": "UNC13C",
  "term_label": "syntaxin-1 binding",
  "gene_name": "Protein unc-13 homolog C"
}